{
  "term_label": "SCF ubiquitin ligase complex",
  "gene": "UniProtKB:Q8N4B4",
  "gene_name": "F-box only protein 39",
  "term_id": "GO:0019005",
  "gene_symbol": "FBXO39"
}